{
  "gene_symbol": "Q5VV11",
  "term_label": "Unknown biological process",
  "term_id": "UNKNOWN:0002",
  "gene_name": "Putative UPF0633 protein ENSP00000303136",
  "gene": "UniProtKB:Q5VV11"
}